{
  "gene": "UniProtKB:E9PQ53",
  "gene_name": "NADH dehydrogenase [ubiquinone] 1 subunit C2, isoform 2",
  "term_id": "GO:0045271",
  "term_label": "respiratory chain complex I",
  "gene_symbol": "NDUFC2-KCTD14"
}